{
  "gene_name": "Tubulin polyglutamylase complex subunit 2",
  "term_id": "UNKNOWN:0002",
  "term_label": "Unknown biological process",
  "gene_symbol": "TPGS2",
  "gene": "UniProtKB:Q68CL5"
}